telomeric D-loop disassembly [GO:0061820] (biological process) References: PMID:10338204, PMID:24012755 Sources: GOC:BHF, GOC:BHF_telomere, GOC:nc Relationships: is a type of telomeric loop disassembly [GO:0090657] Definition: A telomere loop disassembly process that results in the disassembly of telomeric D-loops. A telomeric D-loop is a three-stranded DNA displacement loop that forms at the site where the telomeric 3' single-stranded DNA overhang (formed of the repeat sequence TTAGGG in mammals) is tucked back inside the double-stranded component of telomeric DNA molecule, thus forming a t-loop or telomeric-loop and protecting the chromosome terminus. Regulation: regulated by regulation of telomeric D-loop disassembly [GO:1905838]; negatively regulated by negative regulation of telomeric D-loop disassembly [GO:1905839]; positively regulated by GO:1905840